{
  "gene_name": "Peroxiredoxin-5, mitochondrial",
  "term_id": "GO:0034599",
  "gene": "UniProtKB:P30044",
  "term_label": "cellular response to oxidative stress",
  "gene_symbol": "PRDX5"
}